positive regulation of interleukin-35-mediated signaling pathway [GO:0070760] (biological process) Definition: Any process that increases the rate, frequency or extent of an interleukin-35-mediated signaling pathway. Relationships: is a type of positive regulation of cytokine-mediated signaling pathway [GO:0001961]; is_a regulation of interleukin-35-mediated signaling pathway [GO:0070758]; positively regulates GO:0070757 Also known as: positive regulation of IL-35-mediated signaling pathway, positive regulation of interleukin-35-mediated signalling pathway Sources: GOC:mah